{
  "term_label": "Unknown biological process",
  "gene": "UniProtKB:P34059",
  "term_id": "UNKNOWN:0002",
  "gene_name": "N-acetylgalactosamine-6-sulfatase",
  "gene_symbol": "GALNS"
}